{
  "term_id": "GO:0050839",
  "gene": "UniProtKB:Q9Y5I3",
  "term_label": "cell adhesion molecule binding",
  "gene_name": "Protocadherin alpha-1",
  "gene_symbol": "PCDHA1"
}